{
  "gene": "UniProtKB:A6NGY1",
  "term_label": "Unknown cellular component",
  "gene_symbol": "FRG2C",
  "term_id": "UNKNOWN:0003",
  "gene_name": "Protein FRG2-like-2"
}